negative regulation of translational termination [GO:0045904] (biological process) Definition: Any process that stops, prevents, or reduces the frequency, rate or extent of translational termination. Sources: GOC:go_curators Relationships: is a type of regulation of translational termination [GO:0006449]; is a type of GO:0017148; is a type of negative regulation of protein-containing complex disassembly [GO:0043242]; negatively regulates GO:0006415 Also known as: down regulation of translational termination, down-regulation of translational termination, downregulation of translational termination, inhibition of translational termination